{
  "term_id": "UNKNOWN:0003",
  "gene": "UniProtKB:Q6ZMT9",
  "gene_name": "Death domain-containing protein 1",
  "term_label": "Unknown cellular component",
  "gene_symbol": "DTHD1"
}